{
  "gene_name": "Large ribosomal subunit protein uL29m",
  "gene": "UniProtKB:Q9HD33",
  "term_id": "GO:0032543",
  "gene_symbol": "MRPL47",
  "term_label": "mitochondrial translation"
}